{
  "term_label": "Unknown molecular function",
  "term_id": "UNKNOWN:0001",
  "gene": "UniProtKB:Q7Z5K2",
  "gene_symbol": "WAPL",
  "gene_name": "Wings apart-like protein homolog"
}